{
  "term_label": "DNA damage response",
  "gene": "UniProtKB:Q86WJ1",
  "term_id": "GO:0006974",
  "gene_name": "Chromodomain-helicase-DNA-binding protein 1-like",
  "gene_symbol": "CHD1L"
}